{
  "term_id": "GO:0006493",
  "gene_symbol": "GALNT8",
  "gene": "UniProtKB:Q9NY28",
  "gene_name": "Probable polypeptide N-acetylgalactosaminyltransferase 8",
  "term_label": "protein O-linked glycosylation"
}